{
  "gene_name": "Small nuclear ribonucleoprotein F",
  "gene": "UniProtKB:P62306",
  "term_label": "catalytic step 2 spliceosome",
  "term_id": "GO:0071013",
  "gene_symbol": "SNRPF"
}